acireductone dioxygenase [iron(II)-requiring] activity [GO:0010309] (molecular function) Definition: Catalysis of the reaction: 1,2-dihydroxy-5-(methylthio)pent-1-en-3-one + O2 = 4-methylthio-2-oxobutanoate + formate + H+. Relationships: is a type of oxidoreductase activity, acting on single donors with incorporation of molecular oxygen, incorporation of two atoms of oxygen [GO:0016702] Also known as: 2-hydroxy-3-keto-5-thiomethylpent-1-ene dioxygenase, aci-reductone dioxygenase, acireductone dioxygenase activity, 1,2-dihydroxy-3-keto-5-methylthiopentene dioxygenase activity, acireductone dioxygenase (Fe2+-requiring) activity, 1,2-dihydroxy-5-(methylthio)pent-1-en-3-one:oxygen oxidoreductase (formate-forming), ARD', ARD1, E-2' Sources: EC:1.13.11.54, RHEA:24504